{
  "gene_symbol": "SYCP2L",
  "gene": "UniProtKB:Q5T4T6",
  "gene_name": "Synaptonemal complex protein 2-like",
  "term_id": "UNKNOWN:0001",
  "term_label": "Unknown molecular function"
}